toll-like receptor 15 signaling pathway [GO:0035681] (biological process) Definition: The series of molecular signals initiated by a ligand binding to toll-like receptor 15. Relationships: is a type of cell surface toll-like receptor signaling pathway [GO:0140895] Also known as: TLR15 signaling pathway, toll-like receptor 15 signalling pathway Sources: GOC:pde Regulation: regulated by GO:2000440; negatively regulated by negative regulation of toll-like receptor 15 signaling pathway [GO:2000441]; positively regulated by positive regulation of toll-like receptor 15 signaling pathway [GO:2000442]